{
  "gene": "UniProtKB:P21917",
  "gene_symbol": "DRD4",
  "gene_name": "D(4) dopamine receptor",
  "term_id": "GO:0005886",
  "term_label": "plasma membrane"
}